myelin sheath adaxonal region [GO:0035749] (cellular component) Relationships: is a type of cellular anatomical structure [GO:0110165]; is part of myelin sheath [GO:0043209] References: PMID:20237282 Sources: GOC:BHF Definition: The region of the myelin sheath nearest to the axon.